{
  "gene": "UniProtKB:Q9BZW5",
  "gene_symbol": "TM6SF1",
  "gene_name": "Transmembrane 6 superfamily member 1",
  "term_label": "Unknown molecular function",
  "term_id": "UNKNOWN:0001"
}